defense response by callose deposition in cell wall [GO:0052544] (biological process) Also known as: callose localization in cell wall during defense response, cell wall callose deposition during defense response, cell wall callose localization during defense response, callose deposition in cell wall during defense response Sources: GOC:mtg_pamgo_17jul06 Definition: Any process in which callose is transported to, and/or maintained in, the cell wall during the defense response. Callose is a linear 1,3-beta-d-glucan formed from UDP-glucose and is found in certain plant cell walls. Relationships: is a type of GO:0052482; is a type of defense response by callose deposition [GO:0052542]; is a type of callose deposition in cell wall [GO:0052543]; BFO_0000050 defense response [GO:0006952]